{
  "term_label": "Unknown biological process",
  "gene_name": "Coiled-coil domain-containing protein 6",
  "gene_symbol": "CCDC6",
  "term_id": "UNKNOWN:0002",
  "gene": "UniProtKB:Q16204"
}